{
  "gene_symbol": "STAMBP",
  "term_label": "endosome",
  "gene_name": "STAM-binding protein",
  "term_id": "GO:0005768",
  "gene": "UniProtKB:O95630"
}